{
  "term_label": "GTP binding",
  "gene_name": "ADP-ribosylation factor-like protein 4A",
  "gene": "UniProtKB:P40617",
  "term_id": "GO:0005525",
  "gene_symbol": "ARL4A"
}